4-pyridoxolactonase activity [GO:0047585] (molecular function) Definition: Catalysis of the reaction: 4-pyridoxolactone + H2O = 4-pyridoxate + H+. Also known as: 4-pyridoxolactone lactonohydrolase activity Sources: EC:3.1.1.27, RHEA:14301 Relationships: is a type of carboxylic ester hydrolase activity [GO:0052689]